L-amino acid efflux transmembrane transporter activity [GO:0034639] (molecular function) Sources: GOC:mah Subtypes: threonine efflux transmembrane transporter activity [GO:0015565], L-lysine efflux transmembrane transporter activity [GO:0015661] Definition: Enables the transfer of an L-amino acid from the inside of the cell to the outside of the cell across a membrane. Relationships: is a type of L-amino acid transmembrane transporter activity [GO:0015179]; is a type of efflux transmembrane transporter activity [GO:0015562] Also known as: L-amino acid efflux permease activity, L-amino acid export transporter activity